{
  "term_label": "Unknown molecular function",
  "term_id": "UNKNOWN:0001",
  "gene_symbol": "GRXCR1",
  "gene_name": "Glutaredoxin domain-containing cysteine-rich protein 1",
  "gene": "UniProtKB:A8MXD5"
}